{
  "gene": "UniProtKB:Q9Y6Q3",
  "gene_name": "Zinc finger protein 37 homolog",
  "gene_symbol": "ZFP37",
  "term_label": "regulation of transcription by RNA polymerase II",
  "term_id": "GO:0006357"
}